{
  "gene_symbol": "ZMAT2",
  "term_label": "U4/U6 x U5 tri-snRNP complex",
  "term_id": "GO:0046540",
  "gene": "UniProtKB:Q96NC0",
  "gene_name": "Zinc finger matrin-type protein 2"
}